{
  "gene": "UniProtKB:Q9UNZ2",
  "gene_symbol": "NSFL1C",
  "term_id": "GO:0031468",
  "term_label": "nuclear membrane reassembly",
  "gene_name": "NSFL1 cofactor p47"
}